{
  "gene": "UniProtKB:O95347",
  "term_label": "chromatin",
  "term_id": "GO:0000785",
  "gene_name": "Structural maintenance of chromosomes protein 2",
  "gene_symbol": "SMC2"
}